{
  "gene_symbol": "SNAP91",
  "gene": "UniProtKB:O60641",
  "term_id": "GO:0030136",
  "gene_name": "Clathrin coat assembly protein AP180",
  "term_label": "clathrin-coated vesicle"
}